dopamine beta-monooxygenase activity [GO:0004500] (molecular function) Definition: Catalysis of the reaction: L-ascorbate + dopamine + O2 = (R)-noradrenaline + dehydroascorbate + H2O. Sources: EC:1.14.17.1, RHEA:19117 Also known as: dopamine b-hydroxylase activity, (3,4-dihydroxyphenethylamine)beta-mono-oxygenase activity, 3,4-dihydroxyphenethylamine beta-oxidase activity, 3,4-dihydroxyphenethylamine,ascorbate:oxygen oxidoreductase (beta-hydroxylating), 4-(2-aminoethyl)pyrocatechol beta-oxidase activity, MDBH (membrane-associated dopamine beta-monooxygenase), SDBH (soluble dopamine beta-monooxygenase), dopa beta-hydroxylase activity, dopamine beta-hydroxylase activity, dopamine beta-oxidase activity, dopamine hydroxylase activity, dopamine-B-hydroxylase activity, oxygenase, dopamine beta-mono-, phenylamine beta-hydroxylase activity Relationships: is a type of oxidoreductase activity, acting on paired donors, with incorporation or reduction of molecular oxygen, reduced ascorbate as one donor, and incorporation of one atom of oxygen [GO:0016715]